sculpture element [GO:0043675] (cellular component) Sources: https://doi.org/10.1007/978-3-319-71365-6_3 Definition: The third layer of the sexine. Relationships: is_a cellular anatomical structure [GO:0110165]; is part of sexine [GO:0043673]